{
  "gene": "UniProtKB:P14625",
  "gene_name": "Endoplasmin",
  "gene_symbol": "HSP90B1",
  "term_label": "unfolded protein binding",
  "term_id": "GO:0051082"
}